{
  "gene_symbol": "GVQW3",
  "gene_name": "Protein GVQW3",
  "term_label": "Unknown cellular component",
  "term_id": "UNKNOWN:0003",
  "gene": "UniProtKB:Q3ZCU0"
}